{
  "gene": "UniProtKB:P15085",
  "gene_name": "Carboxypeptidase A1",
  "term_label": "extracellular space",
  "gene_symbol": "CPA1",
  "term_id": "GO:0005615"
}